RNA polymerase II CTD heptapeptide repeat P6 isomerase activity [GO:0140840] (molecular function) Relationships: is a type of RNA polymerase II CTD heptapeptide repeat peptidyl-prolyl isomerase activity [GO:0140838] Also known as: RNA polymerase II C-terminal domain P6 isomerase activity References: PMID:28248323 Definition: Catalysis of the reaction: RNA polymerase II large subunit CTD heptapeptide repeat (consensus YSPTSPS) cis-proline (omega=180) (position 6) = RNA polymerase II large subunit trans-proline (omega=0) (position 6).